{
  "term_id": "GO:0043022",
  "term_label": "ribosome binding",
  "gene_name": "Eukaryotic translation initiation factor 2 subunit 1",
  "gene_symbol": "EIF2S1",
  "gene": "UniProtKB:P05198"
}